{
  "gene": "UniProtKB:A4QPH2",
  "gene_symbol": "PI4KAP2",
  "term_id": "UNKNOWN:0003",
  "term_label": "Unknown cellular component",
  "gene_name": "Putative phosphatidylinositol 4-kinase alpha-like protein P2"
}